{
  "gene": "UniProtKB:Q99880",
  "gene_symbol": "H2BC13",
  "term_label": "extracellular space",
  "gene_name": "Histone H2B type 1-L",
  "term_id": "GO:0005615"
}